{
  "term_label": "cytosol",
  "gene": "UniProtKB:Q8TB92",
  "gene_name": "3-hydroxy-3-methylglutaryl-CoA lyase, cytoplasmic",
  "gene_symbol": "HMGCLL1",
  "term_id": "GO:0005829"
}